{
  "term_id": "UNKNOWN:0002",
  "gene_name": "Small integral membrane protein 21",
  "gene_symbol": "SMIM21",
  "gene": "UniProtKB:Q3B7S5",
  "term_label": "Unknown biological process"
}